branched-chain amino acid catabolic process to alcohol via Ehrlich pathway [GO:0000950] (biological process) Also known as: branched chain family amino acid catabolic process to alcohol via Ehrlich pathway Definition: The chemical reactions and pathways involving the catabolism of branched chain amino acids to produce branched chain alcohols with one carbon less than the starting amino acid. In S. cerevisiae, this is known to occur for leucine, isoleucine, valine, methionine, phenylalanine, tyrosine, or tryptophan. When a branched chain family amino acid, leucine, isoleucine, or valine, is used as the substrate, 3-methylbutanol, 2-methylbutanol, or 2-methylpropanol, respectively, is produced. Often referred to as the Ehrlich pathway, these reactions generally occur during fermentation to produce a variety of alcohols, often collectively referred to as fusel alcohols. Depending on the redox state of the cells, carboxylic acid derivatives may be produced instead of alcohols. References: PMID:18281432 Sources: GOC:krc Relationships: is a type of amino acid catabolic process to alcohol via Ehrlich pathway [GO:0000947]; is a type of branched-chain amino acid catabolic process [GO:0009083]